methylenetetrahydrofolate reductase (ferredoxin) activity [GO:0033738] (molecular function) Also known as: 5,10-methylenetetrahydrofolate reductase activity, 5-methyltetrahydrofolate:ferredoxin oxidoreductase activity Definition: Catalysis of the reaction: 5-methyltetrahydrofolate + oxidized ferredoxin = 5,10-methylenetetrahydrofolate + reduced ferredoxin. Sources: EC:1.5.7.1 Relationships: is a type of GO:0033694